{
  "gene": "UniProtKB:O75845",
  "gene_name": "Lathosterol oxidase",
  "term_id": "GO:0016020",
  "term_label": "membrane",
  "gene_symbol": "SC5D"
}